{
  "term_id": "GO:0005737",
  "term_label": "cytoplasm",
  "gene_name": "Calpastatin",
  "gene_symbol": "CAST",
  "gene": "UniProtKB:P20810"
}